apolipoprotein receptor binding [GO:0034190] (molecular function) Definition: Binding to an apolipoprotein receptor. Subtypes: apolipoprotein A-I receptor binding [GO:0034191] Sources: GOC:BHF, GOC:rl Relationships: is a type of signaling receptor binding [GO:0005102]